{
  "gene_name": "D(2) dopamine receptor",
  "term_id": "GO:0001591",
  "gene": "UniProtKB:P14416",
  "term_label": "dopamine neurotransmitter receptor activity, coupled via Gi/Go",
  "gene_symbol": "DRD2"
}